tubulin complex assembly [GO:0007021] (BP) Definition: The aggregation and bonding together of alpha- and beta-tubulin to form a tubulin heterodimer. Sources: GOC:mah Relationships: is a type of protein-containing complex assembly [GO:0065003] Also known as: tubulin assembly, tubulin folding, tubulin-specific chaperone activity